sphingosine biosynthetic process [GO:0046512] (biological process) Also known as: sphingosine anabolism, sphingosine biosynthesis, sphingosine formation, sphingosine synthesis Relationships: is a type of sphingosine metabolic process [GO:0006670]; is a type of diol biosynthetic process [GO:0034312]; is a type of GO:0046520 Sources: GOC:ma, ISBN:0198506732 Definition: The chemical reactions and pathways resulting in the formation of sphingosine (sphing-4-enine), trans-D-erytho-2-amino-octadec-4-ene-1,3-diol, a long chain amino diol sphingoid base that occurs in most sphingolipids in animal tissues.